pentameric IgM immunoglobulin complex [GO:0071756] (CC) Note: Note that an IgM immunoglobulin complex has the function of antigen binding if a suitable antigen is available. References: PMID:20176268 Sources: GOC:add, ISBN:0781765196 Definition: A circulating form of IgM consisting of a pentamer of IgM core units with a single J chain polypeptide. Relationships: is a type of IgM immunoglobulin complex, circulating [GO:0071754] Also known as: pentameric IgM antibody